{
  "gene": "UniProtKB:Q4AE62",
  "term_id": "GO:0006400",
  "term_label": "tRNA modification",
  "gene_name": "Glycosyltransferase-like domain-containing protein 1",
  "gene_symbol": "GTDC1"
}